{
  "term_label": "mitophagy by internal vacuole formation",
  "gene_name": "Mitochondria-eating protein",
  "gene_symbol": "SPATA18",
  "term_id": "GO:0035695",
  "gene": "UniProtKB:Q8TC71"
}